sorbitol transmembrane transporter activity [GO:0015576] (molecular function) Also known as: glucitol permease activity, glucitol transporter activity, sorbitol permease activity Relationships: is a type of carbohydrate transmembrane transporter activity [GO:0015144]; is a type of polyol transmembrane transporter activity [GO:0015166]; is a type of active transmembrane transporter activity [GO:0022804]; is part of sorbitol transmembrane transport [GO:0015795] Subtypes: GO:0022856 Sources: GOC:ai, ISBN:0198506732 Definition: Enables the transfer of sorbitol from one side of a membrane to the other. Sorbitol, also known as glucitol, is the hexitol derived by the reduction of the aldehyde group of glucose.